{
  "gene": "UniProtKB:O95081",
  "gene_name": "Arf-GAP domain and FG repeat-containing protein 2",
  "term_id": "GO:0005737",
  "gene_symbol": "AGFG2",
  "term_label": "cytoplasm"
}